{
  "gene": "UniProtKB:P56748",
  "gene_name": "Claudin-8",
  "term_id": "GO:0005886",
  "gene_symbol": "CLDN8",
  "term_label": "plasma membrane"
}